{
  "gene": "UniProtKB:P57740",
  "term_label": "post-transcriptional tethering of RNA polymerase II gene DNA at nuclear periphery",
  "term_id": "GO:0000973",
  "gene_name": "Nuclear pore complex protein Nup107",
  "gene_symbol": "NUP107"
}